viral penetration into host nucleus [GO:0075732] (biological process) Definition: The crossing by the virus of the host nuclear membrane, either as naked viral genome or for small viruses as an intact capsid. References: PMID:22929056 Sources: VZ:989 Also known as: viral entry into host nucleus, viral import into host nucleus Relationships: is a type of intracellular transport of virus [GO:0075733] Subtypes: entry of intact viral capsid into host nucleus through nuclear pore complex [GO:0075505], GO:0075506, entry of viral genome into host nucleus via docking of viral capsid to the nuclear pore complex and injection of viral genome [GO:0075507], GO:0075508